dihydroneopterin triphosphate pyrophosphohydrolase activity [GO:0019177] (MF) Definition: Catalysis of the reaction: dihydroneopterin triphosphate = dihydroneopterin phosphate + diphosphate. Sources: RHEA:25302 Relationships: is a type of pyrophosphatase activity [GO:0016462]